{
  "term_label": "regulation of transcription by RNA polymerase II",
  "term_id": "GO:0006357",
  "gene_name": "Zinc finger protein 584",
  "gene": "UniProtKB:Q8IVC4",
  "gene_symbol": "ZNF584"
}